protein glutathionylation [GO:0010731] (biological process) Definition: The protein modification process in which a glutathione molecule is added to a protein amino acid through a disulfide linkage. Also known as: protein amino acid glutathionylation Sources: GOC:BHF, GOC:dph, GOC:rl, GOC:tb Regulation: regulated by regulation of protein glutathionylation [GO:0010732]; positively regulated by positive regulation of protein glutathionylation [GO:0010733]; negatively regulated by negative regulation of protein glutathionylation [GO:0010734] Relationships: is a type of protein modification process [GO:0036211]